{
  "gene_name": "PRAME family member 33",
  "term_id": "GO:0031462",
  "term_label": "Cul2-RING ubiquitin ligase complex",
  "gene_symbol": "PRAMEF33",
  "gene": "UniProtKB:A0A0G2JMD5"
}